positive regulation of sclerotium development [GO:1901924] (biological process) Also known as: up regulation of sclerotium development, up-regulation of sclerotium development, upregulation of sclerotium development, activation of sclerotium development Relationships: is a type of positive regulation of developmental process [GO:0051094]; is a type of GO:1901922; RO_0002213 sclerotium development [GO:1990045] References: PMID:21148914 Sources: GOC:TermGenie, GOC:di Definition: Any process that activates or increases the frequency, rate or extent of sclerotium development.